{
  "gene_symbol": "PLEKHM2",
  "gene": "UniProtKB:Q8IWE5",
  "term_label": "Golgi organization",
  "gene_name": "Pleckstrin homology domain-containing family M member 2",
  "term_id": "GO:0007030"
}